collagen catabolic process [GO:0030574] (biological process) Relationships: is a type of GO:0009056; is a type of collagen metabolic process [GO:0032963] Sources: GOC:mah, ISBN:0815316194 Definition: The proteolytic chemical reactions and pathways resulting in the breakdown of collagen in the extracellular matrix, usually carried out by proteases secreted by nearby cells. Also known as: collagen breakdown, collagen catabolism, collagen degradation Regulation: regulated by GO:0010710; negatively regulated by negative regulation of collagen catabolic process [GO:0010711]; positively regulated by positive regulation of collagen catabolic process [GO:0120158]